{
  "gene_name": "Protein Jade-3",
  "term_id": "GO:0006338",
  "gene": "UniProtKB:Q92613",
  "term_label": "chromatin remodeling",
  "gene_symbol": "JADE3"
}